{
  "gene": "UniProtKB:Q9BTA9",
  "gene_symbol": "WAC",
  "gene_name": "WW domain-containing adapter protein with coiled-coil",
  "term_id": "GO:0010506",
  "term_label": "regulation of autophagy"
}